{
  "gene": "UniProtKB:A0JD36",
  "term_label": "Unknown cellular component",
  "gene_name": "T cell receptor delta variable 2",
  "term_id": "UNKNOWN:0003",
  "gene_symbol": "TRDV2"
}